deoxyribonuclease II activity [GO:0004531] (molecular function) Definition: Catalysis of the endonucleolytic cleavage of DNA to 3'-phosphodinucleotide and 3'-phosphooligonucleotide end products. Sources: EC:3.1.22.1 Also known as: lysosomal DNase II activity, DNase II activity, acid DNase activity, acid deoxyribonuclease activity, deoxyribonucleate 3'-nucleotidohydrolase activity, pancreatic DNase II Relationships: is a type of DNA endonuclease activity, producing 3'-phosphomonoesters [GO:0016889]